ammon gyrus development [GO:0021541] (biological process) Definition: The process whose specific outcome is the progression of the ammon gyrus over time, from its formation to the mature structure. The ammon gyrus, often subdivided into the CA1 and CA3 regions, is one of the two interlocking gyri of the hippocampus that is rich in large pyramidal neurons. Sources: GOC:cls, GOC:dgh, GOC:dph, GOC:jid, GO_REF:0000021 Also known as: Ammon's horn development, cornu ammonis development Relationships: is a type of anatomical structure development [GO:0048856]; is part of hippocampus development [GO:0021766]